{
  "gene_symbol": "KCND2",
  "term_id": "GO:0005250",
  "term_label": "A-type (transient outward) potassium channel activity",
  "gene_name": "Potassium voltage-gated channel subfamily D member 2",
  "gene": "UniProtKB:Q9NZV8"
}